phospholipase D-activating G protein-coupled receptor signaling pathway [GO:0031583] (biological process) Note: This term is intended to cover steps in a GPCR signaling pathway both upstream and downstream of phospholipase D (PLD) activation. References: PMID:11812783, PMID:15924269 Sources: GOC:mah, GOC:signaling Also known as: G-protein signalling, phospholipase D activating pathway, phospholipase D-activating G-protein coupled receptor signaling pathway, activation of phospholipase D activity by G-protein coupled receptor protein signaling pathway Definition: A G protein-coupled receptor signaling pathway in which the signal is transmitted via the activation of phospholipase D (PLD) and a subsequent increase in the intracellular concentration of phosphatidic acid (PA). Relationships: is a type of GO:0007186